{
  "term_label": "Unknown biological process",
  "term_id": "UNKNOWN:0002",
  "gene": "UniProtKB:Q96KC8",
  "gene_name": "DnaJ homolog subfamily C member 1",
  "gene_symbol": "DNAJC1"
}